trypanothione catabolic process [GO:0046207] (biological process) Relationships: is a type of trypanothione metabolic process [GO:0046206]; is a type of glutathione derivative catabolic process [GO:1901686] Sources: GOC:ai Also known as: trypanothione breakdown, trypanothione catabolism, trypanothione degradation Definition: The chemical reactions and pathways resulting in the breakdown of trypanothione (N1,N6,-bis(glutathionyl)spermidine), an essential redox intermediate in intracellular thiol redox regulation which also plays a role in protecting against oxidative stress.